{
  "gene_name": "Probetacellulin",
  "term_id": "GO:0005154",
  "gene_symbol": "BTC",
  "gene": "UniProtKB:P35070",
  "term_label": "epidermal growth factor receptor binding"
}